cell adhesion involved in multi-species biofilm formation [GO:0043710] (biological process) Definition: The attachment of a cell to a solid substrate, via cell adhesion molecules, contributing to the formation of a biofilm composed of microorganisms of different species. Sources: GOC:dph, GOC:jl, GOC:tb Also known as: cell adhesion during multi-species biofilm formation Relationships: is_a cell adhesion involved in biofilm formation [GO:0043708]; is part of multi-species biofilm formation [GO:0044399]